{
  "gene_name": "CCR4-NOT transcription complex subunit 2",
  "term_label": "Unknown molecular function",
  "gene_symbol": "CNOT2",
  "gene": "UniProtKB:Q9NZN8",
  "term_id": "UNKNOWN:0001"
}